{
  "gene_symbol": "JMY",
  "term_label": "positive regulation of apoptotic process",
  "gene_name": "Junction-mediating and -regulatory protein",
  "term_id": "GO:0043065",
  "gene": "UniProtKB:Q8N9B5"
}